{
  "term_label": "metalloendopeptidase inhibitor activity",
  "gene_name": "Testican-3",
  "gene_symbol": "SPOCK3",
  "term_id": "GO:0008191",
  "gene": "UniProtKB:Q9BQ16"
}